{
  "gene": "UniProtKB:O43143",
  "term_label": "helicase activity",
  "term_id": "GO:0004386",
  "gene_symbol": "DHX15",
  "gene_name": "ATP-dependent RNA helicase DHX15"
}